{
  "gene_symbol": "SURF1",
  "term_id": "GO:0033617",
  "gene": "UniProtKB:Q15526",
  "term_label": "mitochondrial respiratory chain complex IV assembly",
  "gene_name": "Surfeit locus protein 1"
}